{
  "gene_symbol": "LAT",
  "term_id": "GO:0036398",
  "gene": "UniProtKB:O43561",
  "gene_name": "Linker for activation of T-cells family member 1",
  "term_label": "TCR signalosome"
}